2-methylbut-2-enoyl-CoA(4-) biosynthetic process [GO:1902194] (BP) Also known as: 2-methylbut-2-enoyl-CoA(4-) anabolism, 2-methylbut-2-enoyl-CoA(4-) biosynthesis, 2-methylbut-2-enoyl-CoA(4-) formation, 2-methylbut-2-enoyl-CoA(4-) synthesis Relationships: is a type of fatty-acyl-CoA biosynthetic process [GO:0046949]; is a type of GO:1902192 References: PMID:15574432 Sources: GOC:TermGenie Definition: The chemical reactions and pathways resulting in the formation of 2-methylbut-2-enoyl-CoA(4-).